{
  "term_label": "Unknown molecular function",
  "gene_symbol": "SASS6",
  "term_id": "UNKNOWN:0001",
  "gene_name": "Spindle assembly abnormal protein 6 homolog",
  "gene": "UniProtKB:Q6UVJ0"
}